{
  "term_label": "Unknown cellular component",
  "gene": "UniProtKB:Q9NWM3",
  "term_id": "UNKNOWN:0003",
  "gene_symbol": "CUEDC1",
  "gene_name": "CUE domain-containing protein 1"
}